guard mother cell differentiation [GO:0010444] (BP) Definition: The process in which a meristemoid acquires the specialized features of a guard mother cell. Sources: GOC:expert_db, GOC:tb Relationships: is a type of plant epidermal cell differentiation [GO:0090627]; is part of stomatal lineage progression [GO:0010440]